{
  "gene": "UniProtKB:Q9Y5R2",
  "term_id": "GO:0005615",
  "term_label": "extracellular space",
  "gene_name": "Matrix metalloproteinase-24",
  "gene_symbol": "MMP24"
}